{
  "gene_name": "Integral membrane protein DGCR2_IDD",
  "term_id": "UNKNOWN:0002",
  "gene": "UniProtKB:P98153",
  "term_label": "Unknown biological process",
  "gene_symbol": "DGCR2"
}